{
  "gene_symbol": "CSAD",
  "gene_name": "Cysteine sulfinic acid decarboxylase",
  "term_label": "cytoplasm",
  "gene": "UniProtKB:Q9Y600",
  "term_id": "GO:0005737"
}